{
  "term_label": "Unknown biological process",
  "term_id": "UNKNOWN:0002",
  "gene_name": "Alpha-1-acid glycoprotein 2",
  "gene_symbol": "ORM2",
  "gene": "UniProtKB:P19652"
}